{
  "gene_symbol": "IL21",
  "gene_name": "Interleukin-21",
  "term_id": "UNKNOWN:0003",
  "term_label": "Unknown cellular component",
  "gene": "UniProtKB:Q9HBE4"
}